{
  "gene_name": "Cryptochrome-1",
  "gene": "UniProtKB:Q16526",
  "term_label": "FAD binding",
  "gene_symbol": "CRY1",
  "term_id": "GO:0071949"
}